{
  "gene_name": "Semaphorin-6A",
  "term_id": "GO:0001755",
  "term_label": "neural crest cell migration",
  "gene_symbol": "SEMA6A",
  "gene": "UniProtKB:Q9H2E6"
}